regulation of mitotic sister chromatid separation [GO:0010965] (biological process) Relationships: is a type of regulation of chromosome separation [GO:1905818]; regulates mitotic sister chromatid separation [GO:0051306] Sources: GOC:dph, GOC:tb Subtypes: regulation of mitotic cell cycle spindle assembly checkpoint [GO:0090266], positive regulation of mitotic sister chromatid separation [GO:1901970], GO:1905822, negative regulation of mitotic sister chromatid separation [GO:2000816] Definition: Any process that modulates the frequency, rate or extent of mitotic sister chromatid separation. Mitotic sister chromatid separation is the process in which sister chromatids are physically detached from each other during mitosis.